{
  "gene_symbol": "IP6K2",
  "term_id": "GO:0032958",
  "term_label": "inositol phosphate biosynthetic process",
  "gene": "UniProtKB:Q9UHH9",
  "gene_name": "Inositol hexakisphosphate kinase 2"
}